cytoskeleton of dendritic spine [GO:0098836] (cellular component) Relationships: is a type of GO:0099571; is part of GO:0043197 Subtypes: actin cytoskeleton of dendritic spine [GO:0098938] Definition: The portion of the cytoskeleton that lies within a dendritic spine. The actin component of this cytoskeleton is involved in spine head remodeling in response to postsynaptic signaling. References: PMID:24854120